{
  "gene": "UniProtKB:Q92828",
  "term_id": "GO:0007015",
  "term_label": "actin filament organization",
  "gene_name": "Coronin-2A",
  "gene_symbol": "CORO2A"
}